{
  "gene_symbol": "PMIS2",
  "gene": "UniProtKB:A0A1W2PS18",
  "gene_name": "Transmembrane protein PMIS2",
  "term_id": "UNKNOWN:0001",
  "term_label": "Unknown molecular function"
}